{
  "gene_name": "Inactive N-acetyllactosaminide alpha-1,3-galactosyltransferase",
  "gene": "UniProtKB:Q4G0N0",
  "term_label": "Unknown biological process",
  "term_id": "UNKNOWN:0002",
  "gene_symbol": "GGTA1"
}